{
  "gene_symbol": "LAYN",
  "gene": "UniProtKB:Q6UX15",
  "term_label": "Unknown biological process",
  "gene_name": "Layilin",
  "term_id": "UNKNOWN:0002"
}